{
  "gene_symbol": "MAGED4",
  "term_id": "UNKNOWN:0001",
  "term_label": "Unknown molecular function",
  "gene_name": "Melanoma-associated antigen D4",
  "gene": "UniProtKB:Q96JG8"
}